isopiperitenone delta-isomerase activity [GO:0050008] (molecular function) Sources: RHEA:21516 Relationships: is a type of GO:0016863 Definition: Catalysis of the reaction: isopiperitenone = piperitenone. Also known as: isopiperitenone D-isomerase activity, isopiperitenone delta8-delta4-isomerase activity